{
  "term_label": "bicellular tight junction",
  "gene": "UniProtKB:Q9Y2L6",
  "gene_symbol": "FRMD4B",
  "term_id": "GO:0005923",
  "gene_name": "FERM domain-containing protein 4B"
}